{
  "gene": "UniProtKB:Q9NWV8",
  "term_id": "GO:0016604",
  "term_label": "nuclear body",
  "gene_name": "BRISC and BRCA1-A complex member 1",
  "gene_symbol": "BABAM1"
}